{
  "term_label": "protein localization to plasma membrane",
  "gene_name": "FYN-binding protein 1",
  "term_id": "GO:0072659",
  "gene": "UniProtKB:O15117",
  "gene_symbol": "FYB1"
}